iron ion transmembrane transport [GO:0034755] (biological process) Subtypes: heme transmembrane transport [GO:0035351], iron import into the mitochondrion [GO:0048250], iron ion import across cell outer membrane [GO:0098706], iron ion import across plasma membrane [GO:0098711], iron-sulfur cluster transmembrane transport [GO:1902497], iron ion export across plasma membrane [GO:1903988] Note: Note that this term is not intended for use in annotating lateral movement within membranes. Also known as: iron ion membrane transport, transmembrane iron transport, ferrous ion transmembrane transport, ferrous iron transmembrane transport, high affinity ferrous ion transmembrane transport, high affinity iron ion transport, high-affinity ferrous ion transmembrane transport, high-affinity iron ion transmembrane transport, high-affinity iron ion transport, iron(2+) transmembrane transport, low affinity iron ion transport, low-affinity iron ion transmembrane transport, low-affinity iron ion transport Regulation: RO_0002211 by regulation of iron ion transmembrane transport [GO:0034759]; negatively regulated by GO:0034760; positively regulated by positive regulation of iron ion transmembrane transport [GO:0034761] Definition: A process in which an iron ion is transported from one side of a membrane to the other by means of some agent such as a transporter or pore. References: PMID:11390404 Sources: GOC:mah Relationships: is a type of GO:0006826; is_a GO:0098655